{
  "gene_name": "Syntaxin-19",
  "gene": "UniProtKB:Q8N4C7",
  "term_id": "GO:0005484",
  "term_label": "SNAP receptor activity",
  "gene_symbol": "STX19"
}